{
  "gene_symbol": "UTY",
  "term_id": "GO:0000978",
  "term_label": "RNA polymerase II cis-regulatory region sequence-specific DNA binding",
  "gene": "UniProtKB:O14607",
  "gene_name": "Histone demethylase UTY"
}